{
  "gene": "UniProtKB:Q7Z4I7",
  "term_label": "cell-cell adhesion",
  "term_id": "GO:0098609",
  "gene_symbol": "LIMS2",
  "gene_name": "LIM and senescent cell antigen-like-containing domain protein 2"
}